{
  "gene": "UniProtKB:P11802",
  "gene_symbol": "CDK4",
  "term_label": "signal transduction",
  "term_id": "GO:0007165",
  "gene_name": "Cyclin-dependent kinase 4"
}